{
  "gene_name": "Consortin",
  "term_label": "plasma membrane",
  "term_id": "GO:0005886",
  "gene_symbol": "CNST",
  "gene": "UniProtKB:Q6PJW8"
}